averantin biosynthetic process [GO:1900763] (biological process) Relationships: is a type of polyketide biosynthetic process [GO:0030639]; is a type of GO:0042181; is a type of phenol-containing compound biosynthetic process [GO:0046189] Definition: The chemical reactions and pathways resulting in the formation of averantin. Also known as: averantin anabolism, averantin biosynthesis, averantin formation, averantin synthesis Sources: GOC:TermGenie, GOC:di